{
  "gene_name": "Protein Mdm4",
  "gene": "UniProtKB:O15151",
  "term_label": "transcription repressor complex",
  "term_id": "GO:0017053",
  "gene_symbol": "MDM4"
}